cardiac pacemaker cell fate commitment [GO:0060927] (biological process) Definition: The commitment of cells to pacemaker cell fates and their capacity to differentiate into pacemaker cells. Pacemaker cells are specialized cardiomyocytes that are responsible for regulating the timing of heart contractions. Sources: GOC:mtg_cardiac_conduct_nov11, GOC:mtg_heart Subtypes: atrioventricular node cell fate commitment [GO:0060929], sinoatrial node cell fate commitment [GO:0060930] Relationships: is a type of GO:0060923; is part of cardiac pacemaker cell differentiation [GO:0060920] Also known as: pacemaker cell fate commitment